{
  "gene_symbol": "HRH2",
  "term_label": "neurotransmitter receptor activity",
  "gene_name": "Histamine H2 receptor",
  "term_id": "GO:0030594",
  "gene": "UniProtKB:P25021"
}